{
  "gene": "UniProtKB:Q9H6F2",
  "term_label": "release of sequestered calcium ion into cytosol by sarcoplasmic reticulum",
  "gene_name": "Trimeric intracellular cation channel type A",
  "term_id": "GO:0014808",
  "gene_symbol": "TMEM38A"
}